{
  "gene_symbol": "FOXO4",
  "gene_name": "Forkhead box protein O4",
  "gene": "UniProtKB:P98177",
  "term_label": "regulation of transcription by RNA polymerase II",
  "term_id": "GO:0006357"
}